{
  "term_id": "GO:1900746",
  "gene_name": "Tetraspanin-32",
  "term_label": "regulation of vascular endothelial growth factor signaling pathway",
  "gene": "UniProtKB:Q96QS1",
  "gene_symbol": "TSPAN32"
}